{
  "term_label": "poly(A) RNA polymerase activity",
  "gene_name": "Poly(A) polymerase gamma",
  "term_id": "GO:1990817",
  "gene_symbol": "PAPOLG",
  "gene": "UniProtKB:Q9BWT3"
}